{
  "term_label": "axoneme",
  "term_id": "GO:0005930",
  "gene_name": "Dynein regulatory complex protein 1",
  "gene_symbol": "DRC1",
  "gene": "UniProtKB:Q96MC2"
}